INO80-type complex [GO:0097346] (cellular component) Definition: A chromatin remodeling protein complex initially purified from S. cerevisiae and containing more than 10 subunits, including the SWR1-related complexes. INO80 (inositol requiring 80)-type complexes have diverse functions, including promoting transcriptional activation and DNA repair. Subtypes: GO:0000812, Ino80 complex [GO:0031011] References: PMID:19355820 Sources: GOC:rb Relationships: is a type of GO:0070603